regulation of acute inflammatory response to non-antigenic stimulus [GO:0002877] (biological process) Definition: Any process that modulates the frequency, rate, or extent of an acute inflammatory response to a non-antigenic stimulus. Relationships: is a type of GO:0002673; regulates acute inflammatory response to non-antigenic stimulus [GO:0002525] Subtypes: negative regulation of acute inflammatory response to non-antigenic stimulus [GO:0002878], positive regulation of acute inflammatory response to non-antigenic stimulus [GO:0002879] Sources: GOC:add